regulation of activated CD8-positive, alpha-beta T cell apoptotic process [GO:1905402] (biological process) Definition: Any process that modulates the frequency, rate or extent of activated CD8-positive, alpha-beta T cell apoptotic process. Relationships: is a type of regulation of T cell apoptotic process [GO:0070232]; regulates activated CD8-positive, alpha-beta T cell apoptotic process [GO:1905397] Also known as: regulation of activated CD8-positive, alpha-beta T lymphocyte apoptotic process, regulation of activated CD8-positive, alpha-beta T-cell apoptotic process, regulation of activated CD8-positive, alpha-beta T-lymphocyte apoptotic process, regulation of activated CD8-positive, alpha-beta T cell apoptosis, regulation of activated CD8-positive, alpha-beta T lymphocyte apoptosis, regulation of activated CD8-positive, alpha-beta T-cell apoptosis, regulation of activated CD8-positive, alpha-beta T-lymphocyte apoptosis Subtypes: negative regulation of activated CD8-positive, alpha-beta T cell apoptotic process [GO:1905403], positive regulation of activated CD8-positive, alpha-beta T cell apoptotic process [GO:1905404] References: PMID:24187568 Sources: GOC:TermGenie, GO_REF:0000058